cyanelle thylakoid lumen [GO:0033114] (CC) Definition: The volume enclosed by a cyanelle thylakoid membrane. Sources: GOC:mah Relationships: is a type of plastid thylakoid lumen [GO:0031978]; is part of cyanelle thylakoid [GO:0009843]